{
  "gene_name": "DNA repair protein RAD50",
  "term_id": "GO:0051880",
  "gene": "UniProtKB:Q92878",
  "term_label": "G-quadruplex DNA binding",
  "gene_symbol": "RAD50"
}